{
  "gene_symbol": "ADAMTS6",
  "term_label": "extracellular matrix organization",
  "term_id": "GO:0030198",
  "gene_name": "A disintegrin and metalloproteinase with thrombospondin motifs 6",
  "gene": "UniProtKB:Q9UKP5"
}